{
  "term_label": "Unknown biological process",
  "gene_symbol": "OR8K1",
  "term_id": "UNKNOWN:0002",
  "gene_name": "Olfactory receptor 8K1",
  "gene": "UniProtKB:Q8NGG5"
}